cyclohexadienyl dehydrogenase activity [GO:0047794] (molecular function) Definition: Catalysis of the reaction: L-arogenate + NAD+ = L-tyrosine + NADH + CO2. Sources: EC:1.3.1.43 Also known as: L-arogenate:NAD(+) oxidoreductase activity, L-arogenate:NAD+ oxidoreductase (decarboxylating), L-arogenate:NAD+ oxidoreductase activity, arogenate dehydrogenase activity, arogenic dehydrogenase activity, pretyrosine dehydrogenase activity Relationships: is a type of GO:0016628